{
  "gene_symbol": "IGLL1",
  "gene_name": "Immunoglobulin lambda-like polypeptide 1",
  "term_label": "immunoglobulin mediated immune response",
  "gene": "UniProtKB:P15814",
  "term_id": "GO:0016064"
}